5-aminovalerate transaminase activity [GO:0047589] (molecular function) Also known as: 5-aminovalerate aminotransferase activity, 5-aminopentanoate:2-oxoglutarate aminotransferase activity, delta-aminovalerate aminotransferase activity, delta-aminovalerate transaminase activity Relationships: is a type of transaminase activity [GO:0008483] Definition: Catalysis of the reaction: 2-oxoglutarate + 5-aminopentanoate = 5-oxopentanoate + L-glutamate. Sources: EC:2.6.1.48, RHEA:10212